positive regulation of pro-B cell differentiation [GO:2000975] (biological process) Also known as: positive regulation of pro-B lymphocyte differentiation, positive regulation of pro-B cell development Relationships: is a type of positive regulation of lymphoid progenitor cell differentiation [GO:1905458]; is a type of regulation of pro-B cell differentiation [GO:2000973]; positively regulates pro-B cell differentiation [GO:0002328] Sources: GOC:obol Definition: Any process that activates or increases the frequency, rate or extent of pro-B cell differentiation.